{
  "term_id": "UNKNOWN:0001",
  "gene_symbol": "PRAMEF9",
  "gene": "UniProtKB:P0DUQ2",
  "term_label": "Unknown molecular function",
  "gene_name": "PRAME family member 9"
}